{
  "gene": "UniProtKB:Q9H0U9",
  "gene_name": "Testis-specific Y-encoded-like protein 1",
  "gene_symbol": "TSPYL1",
  "term_id": "UNKNOWN:0002",
  "term_label": "Unknown biological process"
}